{
  "gene_symbol": "PLA2G4A",
  "gene_name": "Cytosolic phospholipase A2",
  "gene": "UniProtKB:P47712",
  "term_label": "cytosol",
  "term_id": "GO:0005829"
}